aspartate-prephenate aminotransferase activity [GO:0033853] (molecular function) Also known as: prephenate transaminase activity, L-arogenate:oxaloacetate aminotransferase activity, L-aspartate:prephenate aminotransferase activity, PAT, prephenate aspartate aminotransferase activity Definition: Catalysis of the reaction: L-arogenate + oxaloacetate = prephenate + L-aspartate. Relationships: is_a transaminase activity [GO:0008483] Sources: RHEA:20445